{
  "term_label": "MCM complex",
  "gene_name": "DNA replication licensing factor MCM7",
  "term_id": "GO:0042555",
  "gene_symbol": "MCM7",
  "gene": "UniProtKB:P33993"
}